histone H2B deubiquitinase activity [GO:0140936] (molecular function) Definition: A histone deubiquitinase that cleaves ubiquitin from a histone H2B protein to which it is conjugated. Subtypes: histone H2B conserved C-terminal lysine deubiquitinase activity [GO:0140935] Relationships: is a type of histone deubiquitinase activity [GO:0140934] Also known as: histone H2B deubiquitination References: PMID:18206972, PMID:29352077